{
  "term_label": "Unknown cellular component",
  "gene": "UniProtKB:P14859",
  "gene_symbol": "POU2F1",
  "gene_name": "POU domain, class 2, transcription factor 1",
  "term_id": "UNKNOWN:0003"
}